{
  "gene_symbol": "NINL",
  "gene_name": "Ninein-like protein",
  "term_label": "centrosome",
  "term_id": "GO:0005813",
  "gene": "UniProtKB:Q9Y2I6"
}